{
  "term_id": "GO:0043161",
  "gene": "UniProtKB:Q5SWL8",
  "gene_symbol": "PRAMEF19",
  "gene_name": "PRAME family member 19",
  "term_label": "proteasome-mediated ubiquitin-dependent protein catabolic process"
}